cardiolipin dehydrogenase (NAD+) activity [GO:0160241] (molecular function) References: PMID:26338420 Sources: RHEA:81091 Relationships: is a type of oxidoreductase activity, acting on the CH-OH group of donors, NAD or NADP as acceptor [GO:0016616] Definition: Catalysis of the reaction: a cardiolipin + NAD+ = a diphosphatidylglycerone + NADH + H+.